{
  "gene": "UniProtKB:Q9H9Y4",
  "gene_symbol": "GPN2",
  "term_id": "GO:0003924",
  "gene_name": "GPN-loop GTPase 2",
  "term_label": "GTPase activity"
}